convergent extension [GO:0060026] (biological process) Relationships: is_a GO:0002009 Subtypes: convergent extension involved in gastrulation [GO:0060027], convergent extension involved in axis elongation [GO:0060028], convergent extension involved in organogenesis [GO:0060029] Definition: The morphogenetic process in which an epithelium narrows along one axis and lengthens in a perpendicular axis. References: PMID:12062082 Sources: GOC:dgf, GOC:dph